polyamine metabolic process [GO:0006595] (biological process) Sources: ISBN:0198506732 Also known as: polyamine metabolism Subtypes: GO:0006596, polyamine catabolic process [GO:0006598], spermine metabolic process [GO:0008215], spermidine metabolic process [GO:0008216], putrescine metabolic process [GO:0009445], GO:0032917, nor-spermidine metabolic process [GO:0046204], polyamine deacetylation [GO:0106047] Relationships: is a type of biogenic amine metabolic process [GO:0006576] Definition: The chemical reactions and pathways involving polyamines, any organic compound containing two or more amino groups.